{
  "term_id": "GO:0045087",
  "gene_name": "Ret finger protein-like 4A-like protein 1",
  "term_label": "innate immune response",
  "gene": "UniProtKB:F8VTS6",
  "gene_symbol": "RFPL4AL1"
}